{
  "gene_symbol": "ATP5F1EP2",
  "term_id": "GO:0046933",
  "gene_name": "ATP synthase subunit epsilon-like protein, mitochondrial",
  "term_label": "proton-transporting ATP synthase activity, rotational mechanism",
  "gene": "UniProtKB:Q5VTU8"
}